{
  "gene_symbol": "CD164L2",
  "term_label": "Unknown biological process",
  "gene": "UniProtKB:Q6UWJ8",
  "gene_name": "CD164 sialomucin-like 2 protein",
  "term_id": "UNKNOWN:0002"
}